{
  "gene": "UniProtKB:Q9Y4Z2",
  "gene_name": "Neurogenin-3",
  "gene_symbol": "NEUROG3",
  "term_id": "GO:0007423",
  "term_label": "sensory organ development"
}